symbiont-mediated activation of host programmed cell death [GO:0052042] (biological process) Subtypes: GO:0034055, GO:0052151 Relationships: is a type of symbiont-mediated perturbation of host programmed cell death [GO:0052040] Definition: A process in which a symbiont gene product activates host programmed cell death, leading to an increase in the frequency, rate or extent of programmed cell death in the host cell. The host is defined as the larger of the organisms involved in a symbiotic interaction. Also known as: activation by organism of host programmed cell death, activation by organism of programmed cell death in other organism during symbiotic interaction, enhancement of host programmed cell death, enhancement of host programmed cell death by organism, induction by organism of programmed cell death in other organism involved in symbiotic interaction, induction by symbiont of host programmed cell death, positive regulation by symbiont of host programmed cell death, upregulation by symbiont of host programmed cell death, activation by organism of non-apoptotic programmed cell death in other organism, activation by symbiont of host programmed cell death, induction by organism of non-apoptotic programmed cell death in other organism during symbiotic interaction, positive regulation by symbiont of host non-apoptotic programmed cell death, stimulation by symbiont of host programmed cell death, induction by organism of programmed cell death in other organism during symbiotic interaction, induction of non-apoptotic programmed cell death by other organism, pathogenesis Sources: GOC:curators